{
  "gene_name": "Zinc finger protein with KRAB and SCAN domains 3",
  "gene_symbol": "ZKSCAN3",
  "term_id": "GO:0006357",
  "gene": "UniProtKB:Q9BRR0",
  "term_label": "regulation of transcription by RNA polymerase II"
}